{
  "term_label": "Unknown molecular function",
  "gene": "UniProtKB:Q15526",
  "gene_symbol": "SURF1",
  "gene_name": "Surfeit locus protein 1",
  "term_id": "UNKNOWN:0001"
}